cellular response to exogenous dsRNA [GO:0071360] (biological process) Also known as: cellular response to exogenous double-stranded RNA, cellular response to viral dsRNA Definition: Any process that results in a change in state or activity of a cell (in terms of movement, secretion, enzyme production, gene expression, etc.) as a result of an exogenous double-stranded RNA stimulus. Sources: GOC:mah Relationships: is a type of response to exogenous dsRNA [GO:0043330]; is a type of cellular response to dsRNA [GO:0071359]